{
  "term_label": "arginine metabolic process",
  "gene_name": "N(G),N(G)-dimethylarginine dimethylaminohydrolase 1",
  "term_id": "GO:0006525",
  "gene": "UniProtKB:O94760",
  "gene_symbol": "DDAH1"
}